{
  "gene": "UniProtKB:Q9NZ52",
  "term_id": "GO:0006893",
  "term_label": "Golgi to plasma membrane transport",
  "gene_symbol": "GGA3",
  "gene_name": "ADP-ribosylation factor-binding protein GGA3"
}